thyroid-stimulating hormone secretion [GO:0070460] (biological process) Regulation: RO_0002211 by regulation of thyroid-stimulating hormone secretion [GO:2000612]; negatively regulated by GO:2000613; positively regulated by GO:2000614 Relationships: is a type of peptide hormone secretion [GO:0030072] Also known as: TSH secretion, thyroid stimulating hormone secretion Definition: The regulated release of thyroid-stimulating hormone, a peptide hormone that stimulates the activity of the thyroid gland, from secretory granules in the anterior pituitary. Sources: GOC:mah, ISBN:0198506732